{
  "term_id": "GO:0016493",
  "gene_symbol": "CCR3",
  "gene_name": "C-C chemokine receptor type 3",
  "term_label": "C-C chemokine receptor activity",
  "gene": "UniProtKB:P51677"
}